{
  "term_label": "transmembrane transporter activity",
  "gene_symbol": "SLC13A4",
  "gene": "UniProtKB:Q9UKG4",
  "gene_name": "Solute carrier family 13 member 4",
  "term_id": "GO:0022857"
}